{
  "term_id": "GO:0048018",
  "gene": "UniProtKB:Q9BZM4",
  "gene_name": "UL16-binding protein 3",
  "term_label": "receptor ligand activity",
  "gene_symbol": "ULBP3"
}